{
  "gene": "UniProtKB:Q76EJ3",
  "term_label": "antiporter activity",
  "gene_name": "UDP-N-acetylglucosamine_UDP-glucose_GDP-mannose transporter",
  "gene_symbol": "SLC35D2",
  "term_id": "GO:0015297"
}